{
  "gene_symbol": "ZNF763",
  "term_label": "regulation of transcription by RNA polymerase II",
  "term_id": "GO:0006357",
  "gene_name": "Zinc finger protein 763",
  "gene": "UniProtKB:Q0D2J5"
}